{
  "term_label": "extracellular space",
  "gene_symbol": "ZP3",
  "term_id": "GO:0005615",
  "gene_name": "Zona pellucida sperm-binding protein 3",
  "gene": "UniProtKB:P21754"
}